{
  "term_id": "GO:0007186",
  "gene": "UniProtKB:Q96R09",
  "term_label": "G protein-coupled receptor signaling pathway",
  "gene_name": "Olfactory receptor 5B2",
  "gene_symbol": "OR5B2"
}